{
  "gene": "UniProtKB:O76082",
  "gene_symbol": "SLC22A5",
  "term_id": "UNKNOWN:0003",
  "gene_name": "Organic cation_carnitine transporter 2",
  "term_label": "Unknown cellular component"
}